{
  "gene_name": "Alpha-ketoglutarate dehydrogenase component 4",
  "gene_symbol": "KGD4",
  "term_label": "oxoglutarate dehydrogenase complex",
  "gene": "UniProtKB:P82909",
  "term_id": "GO:0045252"
}